cardiac muscle tissue regeneration [GO:0061026] (biological process) Regulation: regulated by regulation of cardiac muscle tissue regeneration [GO:1905178]; negatively regulated by negative regulation of cardiac muscle tissue regeneration [GO:1905179]; positively regulated by positive regulation of cardiac muscle tissue regeneration [GO:1905180] Relationships: is a type of tissue regeneration [GO:0042246] Sources: GOC:dph Definition: The regrowth of cardiac muscle tissue to repair injured or damaged muscle fibers in the postnatal stage.